endocytic heme import into cell [GO:0140421] (biological process) Relationships: is a type of endocytic iron import into cell [GO:0140298]; is a type of heme import into cell [GO:0140420] Also known as: heme assimilation References: PMID:28193844 Definition: The directed movement into cell of externally available heme by receptor-mediated endocytosis.